{
  "gene_symbol": "TACR1",
  "term_id": "GO:0097225",
  "term_label": "sperm midpiece",
  "gene": "UniProtKB:P25103",
  "gene_name": "Substance-P receptor"
}